protein auto-ADP-ribosylation [GO:0070213] (biological process) Relationships: is a type of post-translational protein modification [GO:0043687] Definition: The ADP-ribosylation by a protein of one or more of its own amino acid residues, or residues on an identical protein. Sources: GOC:BHF, GOC:rl Also known as: protein amino acid auto-ADP-ribosylation